T-helper 2 cell cytokine production [GO:0035745] (biological process) Sources: CL:0000546, GOC:BHF Relationships: is a type of CD4-positive, alpha-beta T cell cytokine production [GO:0035743]; is part of GO:0042092 Note: Note that this term is in the subset of terms that should not be used for direct gene product annotation. Instead, select one of the 'regulation' children terms. Definition: Any process that contributes to cytokine production by a T-helper 2 cell. Also known as: Th2 cell cytokine production Regulation: regulated by GO:2000551; negatively regulated by negative regulation of T-helper 2 cell cytokine production [GO:2000552]; positively regulated by GO:2000553